{
  "term_label": "single-stranded DNA helicase activity",
  "gene": "UniProtKB:Q8WVB6",
  "gene_symbol": "CHTF18",
  "gene_name": "Chromosome transmission fidelity protein 18 homolog",
  "term_id": "GO:0017116"
}